{
  "term_label": "Unknown molecular function",
  "gene": "UniProtKB:B2RBV5",
  "gene_name": "MORF4 family associated protein 1 like 2",
  "gene_symbol": "MRFAP1L2",
  "term_id": "UNKNOWN:0001"
}